{
  "term_id": "UNKNOWN:0003",
  "gene_symbol": "HMGCS1",
  "term_label": "Unknown cellular component",
  "gene_name": "Hydroxymethylglutaryl-CoA synthase, cytoplasmic",
  "gene": "UniProtKB:Q01581"
}